{
  "gene": "UniProtKB:Q0IIM8",
  "gene_symbol": "TBC1D8B",
  "gene_name": "TBC1 domain family member 8B",
  "term_id": "GO:0005096",
  "term_label": "GTPase activator activity"
}